mitochondrial tricarboxylic acid transmembrane transport [GO:1990546] (biological process) Subtypes: mitochondrial citrate transmembrane transport [GO:0006843] Definition: The process in which a tricarboxylic acid is transported across a mitochondrial membrane, into or out of the mitochondrion. Relationships: is a type of tricarboxylic acid transmembrane transport [GO:0035674] Sources: GOC:vw